{
  "term_label": "plasma membrane",
  "term_id": "GO:0005886",
  "gene_symbol": "LILRB1",
  "gene": "UniProtKB:Q8NHL6",
  "gene_name": "Leukocyte immunoglobulin-like receptor subfamily B member 1"
}